{
  "term_label": "glutathione transferase activity",
  "gene": "UniProtKB:P09210",
  "gene_name": "Glutathione S-transferase A2",
  "gene_symbol": "GSTA2",
  "term_id": "GO:0004364"
}